{
  "term_label": "single-stranded RNA binding",
  "gene_name": "Endonuclease V",
  "gene_symbol": "ENDOV",
  "term_id": "GO:0003727",
  "gene": "UniProtKB:Q8N8Q3"
}